Ig heavy chain-bound endoplasmic reticulum chaperone complex [GO:0034664] (cellular component) Definition: A protein complex that is located in the endoplasmic reticulum (ER) and is formed by the association of an immunoglobulin heavy chain with the proteins of the ER chaperone complex; the latter include BiP, GRP94; CaBP1, protein disulfide isomerase (PDI), ERdj3, cyclophilin B, ERp72, GRP170, UDP-glucosyltransferase, and SDF2-L1. References: PMID:12475965 Also known as: Ig heavy chain-bound ER chaperone complex, immunoglobulin heavy chain-bound endoplasmic reticulum chaperone complex Relationships: is a type of protein folding chaperone complex [GO:0101031]; is a type of endoplasmic reticulum protein-containing complex [GO:0140534]